{
  "term_label": "heme binding",
  "gene_symbol": "CYP2C18",
  "term_id": "GO:0020037",
  "gene_name": "Cytochrome P450 2C18",
  "gene": "UniProtKB:P33260"
}